16-alpha-hydroxyprogesterone dehydratase activity [GO:0047455] (molecular function) Sources: EC:4.2.1.98, MetaCyc:4.2.1.98-RXN Relationships: is a type of hydro-lyase activity [GO:0016836] Definition: Catalysis of the reaction: 16-alpha-hydroxyprogesterone = H2O + 16-dehydroprogesterone. Also known as: hydroxyprogesterone dehydroxylase activity, 16-alpha-dehydroxylase activity, 16-alpha-hydroxyprogesterone dehydroxylase activity, 16-dehydroprogesterone hydratase activity, 16alpha-dehydroxylase activity, 16alpha-hydroxyprogesterone dehydratase activity, 16alpha-hydroxyprogesterone dehydroxylase activity, 16alpha-hydroxyprogesterone hydro-lyase (16,17-didehydroprogesterone-forming), 16alpha-hydroxyprogesterone hydro-lyase activity